positive regulation of timing of exogen [GO:0051888] (biological process) Relationships: is a type of GO:0048818; is a type of regulation of timing of exogen [GO:0051887]; positively regulates exogen [GO:0042638] Also known as: activation of exogen, stimulation of exogen, positive regulation of exogen, up regulation of exogen, up-regulation of exogen, upregulation of exogen Definition: Any process that activates or increases the frequency, rate or extent of timing of exogen, the shedding phase of the hair cycle. Sources: GOC:ai, GOC:pr